{
  "term_id": "GO:0010972",
  "gene_symbol": "WEE1",
  "term_label": "negative regulation of G2/M transition of mitotic cell cycle",
  "gene_name": "Wee1-like protein kinase",
  "gene": "UniProtKB:P30291"
}